{
  "term_id": "GO:0016203",
  "gene_name": "Dystroglycan 1",
  "term_label": "muscle attachment",
  "gene": "UniProtKB:Q14118",
  "gene_symbol": "DAG1"
}